aplanospore formation [GO:0075289] (biological process) Regulation: RO_0002211 by regulation of aplanospore formation [GO:0075290]; positively regulated by GO:0075291; negatively regulated by negative regulation of aplanospore formation [GO:0075292] Sources: GOC:pamgo_curators Relationships: is a type of sporangiospore formation [GO:0034300] Definition: The process in which a nonmotile, asexual spore is formed within a cell in certain algae and fungi (commonly in the Phycomycetes), the wall of aplanospore is distinct from that of the parent cell.